{
  "term_label": "neuron projection",
  "term_id": "GO:0043005",
  "gene": "UniProtKB:Q99463",
  "gene_name": "Putative neuropeptide Y receptor type 6",
  "gene_symbol": "NPY6R"
}